{
  "gene_symbol": "VAV1",
  "term_label": "immune response-regulating cell surface receptor signaling pathway",
  "gene": "UniProtKB:P15498",
  "gene_name": "Proto-oncogene vav",
  "term_id": "GO:0002768"
}